alkanesulfonate binding [GO:0043210] (molecular function) Relationships: is_a anion binding [GO:0043168]; is a type of organic acid binding [GO:0043177]; is a type of sulfur compound binding [GO:1901681] Subtypes: GO:0030977 Definition: Binding to alkanesulfonates, the anion of alkanesulfonic acids, sulfonic acid derivatives containing an aliphatic hydrocarbon group. Sources: GOC:mlg